{
  "gene": "UniProtKB:Q93088",
  "gene_name": "Betaine--homocysteine S-methyltransferase 1",
  "term_label": "cytosol",
  "gene_symbol": "BHMT",
  "term_id": "GO:0005829"
}